{
  "gene": "UniProtKB:Q96NB2",
  "term_id": "GO:0140300",
  "gene_name": "Sideroflexin-2",
  "gene_symbol": "SFXN2",
  "term_label": "serine import into mitochondrion"
}